{
  "term_id": "GO:0035023",
  "gene_symbol": "EPS8",
  "term_label": "regulation of Rho protein signal transduction",
  "gene": "UniProtKB:Q12929",
  "gene_name": "Epidermal growth factor receptor kinase substrate 8"
}